{
  "term_id": "GO:0016303",
  "gene_name": "Phosphatidylinositol 4,5-bisphosphate 3-kinase catalytic subunit alpha isoform",
  "term_label": "1-phosphatidylinositol-3-kinase activity",
  "gene": "UniProtKB:P42336",
  "gene_symbol": "PIK3CA"
}